{
  "gene": "UniProtKB:Q96B23",
  "term_id": "GO:0061630",
  "gene_name": "Protein ARK2N",
  "gene_symbol": "ARK2N",
  "term_label": "ubiquitin protein ligase activity"
}